{
  "term_label": "voltage-gated monoatomic ion channel activity",
  "gene": "UniProtKB:Q4KMQ2",
  "gene_symbol": "ANO6",
  "term_id": "GO:0005244",
  "gene_name": "Anoctamin-6"
}